{
  "term_label": "nucleosome",
  "gene_name": "Core histone macro-H2A.2",
  "term_id": "GO:0000786",
  "gene_symbol": "MACROH2A2",
  "gene": "UniProtKB:Q9P0M6"
}